regulation of androgen secretion [GO:2000834] (biological process) Subtypes: negative regulation of androgen secretion [GO:2000835], GO:2000836 Sources: GOC:sl Relationships: is a type of regulation of steroid hormone secretion [GO:2000831]; regulates androgen secretion [GO:0035935] Definition: Any process that modulates the frequency, rate or extent of androgen secretion.